{
  "gene_symbol": "LAT2",
  "gene": "UniProtKB:Q9GZY6",
  "gene_name": "Linker for activation of T-cells family member 2",
  "term_label": "calcium-mediated signaling",
  "term_id": "GO:0019722"
}